glossopharyngeal nerve maturation [GO:0021614] (biological process) Relationships: is_a cranial nerve maturation [GO:0021605]; is part of GO:0021563 Also known as: CN IX maturation Definition: A developmental process, independent of morphogenetic (shape) change, that is required for the glossopharyngeal nerve to attain its fully functional state. Various sensory and motor branches of the glossopharyngeal nerve supply nerve connections to the pharynx and back of the tongue. The branchial motor component contains motor fibers that innervate muscles that elevate the pharynx and larynx, and the tympanic branch supplies parasympathetic fibers to the otic ganglion. Sources: GOC:cls, GOC:dgh, GOC:dph, GOC:jid, GO_REF:0000021